protein sumoylation [GO:0016925] (biological process) References: PMID:11265250 Sources: GOC:jl Subtypes: protein autosumoylation [GO:1990466] Definition: The process in which a SUMO protein (small ubiquitin-related modifier) is conjugated to a target protein via an isopeptide bond between the carboxy-terminus of SUMO with an epsilon-amino group of a lysine residue of the target protein. Also known as: SUMO-protein conjugation, protein sumolation, small ubiquitin-related protein 1 conjugation, sumoylation, Smt3-protein conjugation, Smt3p-protein conjugation Regulation: regulated by regulation of protein sumoylation [GO:0033233]; negatively regulated by GO:0033234; positively regulated by positive regulation of protein sumoylation [GO:0033235] Relationships: is_a peptidyl-lysine modification [GO:0018205]; is a type of GO:0032446